{
  "gene_symbol": "KIR2DL5A",
  "term_id": "GO:0004888",
  "term_label": "transmembrane signaling receptor activity",
  "gene": "UniProtKB:Q8N109",
  "gene_name": "Killer cell immunoglobulin-like receptor 2DL5A"
}